{
  "gene_symbol": "RGL2",
  "gene_name": "Ral guanine nucleotide dissociation stimulator-like 2",
  "term_label": "Unknown cellular component",
  "term_id": "UNKNOWN:0003",
  "gene": "UniProtKB:O15211"
}